{
  "gene_name": "NUAK family SNF1-like kinase 1",
  "gene": "UniProtKB:O60285",
  "gene_symbol": "NUAK1",
  "term_label": "Unknown cellular component",
  "term_id": "UNKNOWN:0003"
}